{
  "term_label": "very-low-density lipoprotein particle",
  "gene_symbol": "APOC1",
  "gene": "UniProtKB:P02654",
  "term_id": "GO:0034361",
  "gene_name": "Apolipoprotein C-I"
}